{
  "term_label": "serine-type peptidase activity",
  "term_id": "GO:0008236",
  "gene_name": "Serine protease 55",
  "gene": "UniProtKB:Q6UWB4",
  "gene_symbol": "PRSS55"
}